{
  "gene": "UniProtKB:Q6ZSY5",
  "term_id": "GO:0000164",
  "term_label": "protein phosphatase type 1 complex",
  "gene_symbol": "PPP1R3F",
  "gene_name": "Protein phosphatase 1 regulatory subunit 3F"
}